{
  "term_label": "cytosol",
  "term_id": "GO:0005829",
  "gene": "UniProtKB:P08319",
  "gene_symbol": "ADH4",
  "gene_name": "All-trans-retinol dehydrogenase [NAD(+)] ADH4"
}